{
  "gene": "UniProtKB:Q15910",
  "gene_symbol": "EZH2",
  "term_id": "GO:0031507",
  "term_label": "heterochromatin formation",
  "gene_name": "Histone-lysine N-methyltransferase EZH2"
}